{
  "gene": "UniProtKB:Q6ZQV5",
  "term_id": "UNKNOWN:0001",
  "gene_symbol": "ZNF788P",
  "gene_name": "Putative KRAB domain-containing protein ZNF788",
  "term_label": "Unknown molecular function"
}